{
  "term_label": "mitotic DNA damage checkpoint signaling",
  "gene_symbol": "CHEK2",
  "gene": "UniProtKB:O96017",
  "gene_name": "Serine_threonine-protein kinase Chk2",
  "term_id": "GO:0044773"
}